blood microparticle formation [GO:0072564] (biological process) Subtypes: endothelial microparticle formation [GO:0072565] Relationships: is a type of cellular component organization [GO:0016043]; is a type of GO:0048646 References: PMID:16373184 Sources: GOC:BHF, GOC:mah Also known as: microparticle generation, microparticle release Definition: The cellular component organization process in which microparticles bud off from a parent cell. A microparticle is a phospholipid microvesicle that is derived from any of several cell types, such as platelets, blood cells, endothelial cells, or others, and contains membrane receptors as well as other proteins characteristic of the parental cell. Regulation: regulated by GO:2000332; negatively regulated by GO:2000333; positively regulated by positive regulation of blood microparticle formation [GO:2000334]